{
  "gene_symbol": "MOG",
  "term_id": "GO:0001817",
  "gene_name": "Myelin-oligodendrocyte glycoprotein",
  "gene": "UniProtKB:Q16653",
  "term_label": "regulation of cytokine production"
}